{
  "gene": "UniProtKB:Q99814",
  "gene_symbol": "EPAS1",
  "term_id": "GO:0001974",
  "gene_name": "Endothelial PAS domain-containing protein 1",
  "term_label": "blood vessel remodeling"
}